granal stacked thylakoid [GO:0009515] (cellular component) Definition: Appressed thylakoid membranes that are part of a granum (stacked regions). A characteristic of these appressed regions is the preferential localization of photosystem II. Sources: GOC:lr Also known as: chloroplast stacked thylakoid Relationships: is a type of GO:0009534; is part of granum [GO:0009542]